fibroblast growth factor receptor signaling pathway involved in mammary gland specification [GO:0060595] (BP) Relationships: is_a GO:0008543; is part of mammary gland specification [GO:0060594] Definition: The series of molecular signals initiated by binding of a fibroblast growth factor to its receptor on the surface of al cell in the epidermis resulting in the formation of the mammary line. The mammary line is a ridge of epidermal cells that will form the mammary placodes. References: PMID:16168142 Sources: GOC:dph Also known as: fibroblast growth factor receptor signalling pathway involved in mammary gland specification